{
  "term_id": "GO:0099558",
  "gene": "UniProtKB:Q86Z23",
  "gene_symbol": "C1QL4",
  "term_label": "maintenance of synapse structure",
  "gene_name": "Complement C1q-like protein 4"
}